{
  "gene_symbol": "DSCR4",
  "term_label": "Unknown cellular component",
  "gene": "UniProtKB:P56555",
  "term_id": "UNKNOWN:0003",
  "gene_name": "Down syndrome critical region protein 4"
}